{
  "gene_symbol": "SNAPIN",
  "gene_name": "SNARE-associated protein Snapin",
  "term_label": "BLOC-1 complex",
  "term_id": "GO:0031083",
  "gene": "UniProtKB:O95295"
}